{
  "gene": "UniProtKB:Q9H0R1",
  "gene_symbol": "AP5M1",
  "gene_name": "AP-5 complex subunit mu-1",
  "term_label": "Unknown molecular function",
  "term_id": "UNKNOWN:0001"
}